L-alanine:proton antiporter activity [GO:0140407] (molecular function) Relationships: is a type of proton transmembrane transporter activity [GO:0015078]; is_a L-alanine transmembrane transporter activity [GO:0015180]; is a type of amino acid:monoatomic cation antiporter activity [GO:0140848] Definition: Enables the transfer of a solute or solutes from one side of a membrane to the other according to the reaction: H+(out) + L-alanine(in) = H+(in) + L-alanine(out). References: PMID:26073055, PMID:31591285